phosphatidylinositol-5-phosphate phosphatase activity [GO:0102091] (MF) Relationships: is a type of phosphatidylinositol phosphate 5-phosphatase activity [GO:0034595]; is a type of phosphatidylinositol monophosphate phosphatase activity [GO:0052744] Also known as: phosphatidylinositol-5-phosphate 5-phosphatase activity Definition: Catalysis of the reaction: a 1,2-diacyl-sn-glycero-3-phospho-(1D-myo-inositol-5-phosphate) + H2O = a 1,2-diacyl-sn-glycero-3-phospho-(1D-myo-inositol) + phosphate. References: PMID:12878591 Sources: RHEA:41147